negative thymic T cell selection [GO:0045060] (biological process) Also known as: negative thymic T lymphocyte selection, negative thymic T-cell selection, negative thymic T-lymphocyte selection References: PMID:12414722 Sources: ISBN:0781735149 Relationships: is a type of negative T cell selection [GO:0043383]; is a type of thymic T cell selection [GO:0045061] Definition: The process of elimination of immature T cells in the thymus which react strongly with self-antigens.